{
  "term_label": "chromatin remodeling",
  "term_id": "GO:0006338",
  "gene": "UniProtKB:Q17R98",
  "gene_symbol": "ZNF827",
  "gene_name": "Zinc finger protein 827"
}